{
  "gene": "UniProtKB:Q96A44",
  "gene_name": "SPRY domain-containing SOCS box protein 4",
  "term_label": "cytosol",
  "gene_symbol": "SPSB4",
  "term_id": "GO:0005829"
}